{
  "term_label": "Unknown molecular function",
  "gene": "UniProtKB:Q4VC44",
  "term_id": "UNKNOWN:0001",
  "gene_name": "FLYWCH-type zinc finger-containing protein 1",
  "gene_symbol": "FLYWCH1"
}